{
  "term_id": "GO:0005085",
  "term_label": "guanyl-nucleotide exchange factor activity",
  "gene_name": "FYVE, RhoGEF and PH domain-containing protein 2",
  "gene_symbol": "FGD2",
  "gene": "UniProtKB:Q7Z6J4"
}